{
  "gene_symbol": "AVPR2",
  "term_id": "GO:0045907",
  "gene_name": "Vasopressin V2 receptor",
  "gene": "UniProtKB:P30518",
  "term_label": "positive regulation of vasoconstriction"
}